{
  "term_id": "UNKNOWN:0003",
  "term_label": "Unknown cellular component",
  "gene_symbol": "MFAP3",
  "gene": "UniProtKB:P55082",
  "gene_name": "Microfibril-associated glycoprotein 3"
}